{
  "term_label": "Unknown molecular function",
  "term_id": "UNKNOWN:0001",
  "gene_name": "Sialate:O-sulfotransferase 1",
  "gene": "UniProtKB:Q658N2",
  "gene_symbol": "WSCD1"
}